N-methyl-2-oxoglutaramate hydrolase activity [GO:0050130] (molecular function) Sources: EC:3.5.1.36, RHEA:24108 Relationships: is a type of GO:0016811 Definition: Catalysis of the reaction: N-methyl-2-oxoglutaramate + H2O = 2-oxoglutarate + methylammonium. Also known as: 5-hydroxy-N-methylpyroglutamate synthase activity, N-methyl-2-oxoglutaramate methylamidohydrolase activity